{
  "term_label": "urea cycle",
  "term_id": "GO:0000050",
  "gene_symbol": "ARG1",
  "gene": "UniProtKB:P05089",
  "gene_name": "Arginase-1"
}